type II pneumocyte differentiation [GO:0060510] (biological process) Definition: The process in which a relatively unspecialized cell acquires specialized features of a type II pneumocyte. A type II pneumocyte is a surfactant secreting cell that contains abundant cytoplasm containing numerous lipid-rich multilamellar bodies. Sources: GOC:dph, GOC:mtg_lung, ISBN:0721662544 Relationships: is a type of GO:0061140 Also known as: great alveolar cell differentiation, granular pneumocyte differentiation, large alveolar cell differentiation